{
  "term_id": "GO:0016020",
  "term_label": "membrane",
  "gene_symbol": "AMIGO3",
  "gene_name": "Amphoterin-induced protein 3",
  "gene": "UniProtKB:Q86WK7"
}